{
  "term_label": "Unknown cellular component",
  "term_id": "UNKNOWN:0003",
  "gene": "UniProtKB:Q5VT03",
  "gene_name": "NUT family member 2D",
  "gene_symbol": "NUTM2D"
}